negative regulation of interleukin-17-mediated signaling pathway [GO:1903882] (biological process) References: PMID:20054338 Sources: GOC:TermGenie, GOC:krc, GO_REF:0000058 Relationships: is a type of negative regulation of cytokine-mediated signaling pathway [GO:0001960]; is a type of GO:1903881; RO_0002212 interleukin-17-mediated signaling pathway [GO:0097400] Definition: Any process that stops, prevents or reduces the frequency, rate or extent of interleukin-17-mediated signaling pathway. Also known as: down regulation of IL-17-mediated signaling pathway, down regulation of IL-17-mediated signalling pathway, down regulation of interleukin-17-mediated signaling pathway, down regulation of interleukin-17-mediated signalling pathway, down-regulation of IL-17-mediated signaling pathway, down-regulation of IL-17-mediated signalling pathway, down-regulation of interleukin-17-mediated signaling pathway, down-regulation of interleukin-17-mediated signalling pathway, downregulation of IL-17-mediated signaling pathway, downregulation of IL-17-mediated signalling pathway, downregulation of interleukin-17-mediated signaling pathway, downregulation of interleukin-17-mediated signalling pathway, negative regulation of IL-17-mediated signaling pathway, negative regulation of IL-17-mediated signalling pathway, negative regulation of interleukin-17-mediated signalling pathway, inhibition of IL-17-mediated signaling pathway, inhibition of IL-17-mediated signalling pathway, inhibition of interleukin-17-mediated signaling pathway, inhibition of interleukin-17-mediated signalling pathway